seed growth [GO:0080112] (biological process) Regulation: RO_0002211 by regulation of seed growth [GO:0080113] Sources: GOC:dhl, PO:0009010 Definition: The increase in size or mass of a seed. A seed is a propagating organ formed in the reproductive cycle of a spermatophyte, derived from the ovule and enclosing an embryo. Relationships: is a type of GO:0048589; is part of seed development [GO:0048316]